{
  "term_id": "GO:0005669",
  "gene": "UniProtKB:Q6P1X5",
  "term_label": "transcription factor TFIID complex",
  "gene_symbol": "TAF2",
  "gene_name": "Transcription initiation factor TFIID subunit 2"
}